{
  "term_label": "RNA polymerase II transcription regulatory region sequence-specific DNA binding",
  "term_id": "GO:0000977",
  "gene": "UniProtKB:P52736",
  "gene_symbol": "ZNF133",
  "gene_name": "Zinc finger protein 133"
}